translation initiation ternary complex [GO:0044207] (cellular component) Also known as: translation initiation (ternary) complex, Met-tRNA/eIF2.GTP ternary complex Sources: GOC:jl Definition: A ribonucleoprotein complex that contains aminoacylated initiator methionine tRNA, GTP, and initiation factor 2 (either eIF2 in eukaryotes, or IF2 in prokaryotes). In prokaryotes, fMet-tRNA (initiator) is used rather than Met-tRNA (initiator). Relationships: is a type of ribonucleoprotein complex [GO:1990904]; is part of GO:0005737